{
  "gene_symbol": "SLC19A1",
  "term_id": "UNKNOWN:0002",
  "term_label": "Unknown biological process",
  "gene": "UniProtKB:P41440",
  "gene_name": "Reduced folate transporter"
}